{
  "term_id": "GO:0032153",
  "gene_symbol": "SEPTIN2",
  "term_label": "cell division site",
  "gene": "UniProtKB:Q15019",
  "gene_name": "Septin-2"
}